{
  "gene": "UniProtKB:Q6UXX9",
  "gene_name": "R-spondin-2",
  "gene_symbol": "RSPO2",
  "term_id": "GO:0090263",
  "term_label": "positive regulation of canonical Wnt signaling pathway"
}